{
  "gene_name": "Farnesyl pyrophosphate synthase",
  "term_id": "GO:0005737",
  "gene_symbol": "FDPS",
  "term_label": "cytoplasm",
  "gene": "UniProtKB:P14324"
}